peptide hormone receptor binding [GO:0051428] (molecular function) Definition: Binding to a receptor for a peptide hormone. Sources: GOC:ai Also known as: polypeptide hormone receptor binding Relationships: is a type of hormone receptor binding [GO:0051427] Subtypes: gonadotropin-releasing hormone receptor binding [GO:0031530], GO:0031531, corticotropin-releasing hormone receptor binding [GO:0051429], adipokinetic hormone receptor binding [GO:0097005]